{
  "term_id": "UNKNOWN:0001",
  "gene_name": "T-cell surface glycoprotein CD8 beta-2 chain",
  "gene_symbol": "CD8B2",
  "term_label": "Unknown molecular function",
  "gene": "UniProtKB:A6NJW9"
}